{
  "gene_symbol": "PSMB8",
  "term_label": "nucleus",
  "term_id": "GO:0005634",
  "gene_name": "Proteasome subunit beta type-8",
  "gene": "UniProtKB:P28062"
}